plastid inheritance [GO:0009665] (biological process) Definition: The partitioning of plastids between daughter cells at cell division. Sources: GOC:mah Relationships: is a type of plastid organization [GO:0009657]; is a type of organelle inheritance [GO:0048308]